{
  "gene": "UniProtKB:P41162",
  "term_id": "GO:0005634",
  "gene_symbol": "ETV3",
  "gene_name": "ETS translocation variant 3",
  "term_label": "nucleus"
}